inositol-1,3,4,5,6-pentakisphosphate 3-phosphatase activity [GO:0030351] (molecular function) Sources: RHEA:77143 Relationships: is a type of inositol pentakisphosphate phosphatase activity [GO:0052827] Definition: Catalysis of the reaction: 1D-myo-inositol 1,3,4,5,6-pentakisphosphate + H2O = 1D-myo-inositol 1,4,5,6-tetrakisphosphate + phosphate.